{
  "term_id": "UNKNOWN:0001",
  "term_label": "Unknown molecular function",
  "gene_name": "Putative CNGA1-overlapping antisense gene protein",
  "gene": "UniProtKB:Q8IZM0",
  "gene_symbol": "Q8IZM0"
}